lysophospholipid transport [GO:0051977] (biological process) Sources: GOC:ai Relationships: is a type of phospholipid transport [GO:0015914]; is a type of GO:1901264 Definition: The directed movement of phospholipids into, out of or within a cell, or between cells, by means of some agent such as a transporter or pore. A lysophospholipid is a phospholipid that lacks one of its fatty acyl chains; it is an intermediate formed during digestion of dietary and biliary phospholipids. Subtypes: lysophospholipid translocation [GO:0140329]